{
  "gene_name": "DnaJ homolog subfamily A member 3, mitochondrial",
  "term_id": "GO:0005739",
  "gene": "UniProtKB:Q96EY1",
  "gene_symbol": "DNAJA3",
  "term_label": "mitochondrion"
}